regulation of extrinsic apoptotic signaling pathway in absence of ligand [GO:2001239] (biological process) Sources: GOC:mtg_apoptosis Relationships: is a type of GO:2001236; regulates extrinsic apoptotic signaling pathway in absence of ligand [GO:0097192] Definition: Any process that modulates the frequency, rate or extent of extrinsic apoptotic signaling pathway in absence of ligand. Subtypes: negative regulation of extrinsic apoptotic signaling pathway in absence of ligand [GO:2001240], positive regulation of extrinsic apoptotic signaling pathway in absence of ligand [GO:2001241] Also known as: regulation of extrinsic apoptotic signalling pathway in absence of ligand, regulation of extrinsic apoptosis in absence of ligand, regulation of dependence receptor signaling pathway